endocannabinoid signaling pathway involved in trans-synaptic signaling [GO:1905129] (biological process) References: PMID:23040807 Sources: GOC:TermGenie, GO_REF:0000060 Relationships: is a type of endocannabinoid signaling pathway [GO:0071926]; is part of GO:0099542 Subtypes: endocannabinoid signaling pathway involved in retrograde trans-synaptic signaling [GO:1905197] Also known as: endocannabinoid signalling pathway involved in trans-synaptic signaling by endocannabinoid Definition: Any endocannabinoid signaling pathway that is involved in trans-synaptic signaling by endocannabinoid.